{
  "gene": "UniProtKB:Q15418",
  "term_label": "positive regulation of DNA-templated transcription",
  "gene_symbol": "RPS6KA1",
  "term_id": "GO:0045893",
  "gene_name": "Ribosomal protein S6 kinase alpha-1"
}